anther dehiscence [GO:0009901] (biological process) Sources: GOC:tb Regulation: regulated by GO:0120194; positively regulated by positive regulation of anther dehiscence [GO:0120195]; RO_0002212 by negative regulation of anther dehiscence [GO:0120196] Definition: The dehiscence of an anther to release the pollen grains contained within it. Relationships: is_a dehiscence [GO:0009900]; is part of anther development [GO:0048653]